{
  "gene_name": "Stromal membrane-associated protein 1",
  "gene": "UniProtKB:Q8IYB5",
  "term_label": "regulation of clathrin-dependent endocytosis",
  "gene_symbol": "SMAP1",
  "term_id": "GO:2000369"
}